{
  "term_id": "GO:0008046",
  "term_label": "axon guidance receptor activity",
  "gene_symbol": "L1CAM",
  "gene": "UniProtKB:P32004",
  "gene_name": "Neural cell adhesion molecule L1"
}